Toc complex [GO:0010006] (cellular component) Definition: Protein translocon complex at the chloroplast outer membrane. Relationships: is_a membrane protein complex [GO:0098796]; is part of chloroplast outer membrane [GO:0009707] References: PMID:10646606